{
  "gene_name": "HIG1 domain family member 1B",
  "gene": "UniProtKB:Q9P298",
  "gene_symbol": "HIGD1B",
  "term_label": "mitochondrial respirasome assembly",
  "term_id": "GO:0097250"
}